lipopolysaccharide N-acetylmannosaminouronosyltransferase activity [GO:0047241] (molecular function) Definition: Catalysis of the reaction: lipopolysaccharide + UDP-N-acetylmannosaminouronate = N-acetyl-beta-D-mannosaminouronosyl-1,4-lipopolysaccharide + UDP. Sources: RHEA:28366 Also known as: LPS N-acetylmannosaminouronosyltransferase activity, ManNAcA transferase activity, UDP-N-acetyl-beta-D-mannosaminouronate:lipopolysaccharide N-acetyl-beta-D-mannosaminouronosyltransferase activity, uridine diphosphoacetylmannosaminuronate-acetylglucosaminylpyrophosphorylundecaprenol acetylmannosaminuronosyltransferase activity Relationships: is a type of alpha-1,2-mannosyltransferase activity [GO:0000026]; is a type of UDP-glycosyltransferase activity [GO:0008194]